{
  "gene": "UniProtKB:Q9NV66",
  "term_label": "Unknown molecular function",
  "gene_symbol": "TYW1",
  "term_id": "UNKNOWN:0001",
  "gene_name": "S-adenosyl-L-methionine-dependent tRNA 4-demethylwyosine synthase TYW1"
}